{
  "term_id": "GO:0007268",
  "term_label": "chemical synaptic transmission",
  "gene_name": "Disks large homolog 4",
  "gene": "UniProtKB:P78352",
  "gene_symbol": "DLG4"
}